{
  "term_label": "Unknown molecular function",
  "gene": "UniProtKB:Q6P1L5",
  "term_id": "UNKNOWN:0001",
  "gene_name": "Protein FAM117B",
  "gene_symbol": "FAM117B"
}